{
  "gene_name": "Histone-lysine N-methyltransferase EZH1",
  "gene_symbol": "EZH1",
  "gene": "UniProtKB:Q92800",
  "term_label": "chromatin binding",
  "term_id": "GO:0003682"
}